{
  "term_id": "GO:0045494",
  "gene": "UniProtKB:Q9P0W8",
  "gene_name": "Spermatogenesis-associated protein 7",
  "gene_symbol": "SPATA7",
  "term_label": "photoreceptor cell maintenance"
}